{
  "gene_name": "Transmembrane emp24 domain-containing protein 6",
  "gene": "UniProtKB:Q8WW62",
  "term_id": "GO:0005793",
  "term_label": "endoplasmic reticulum-Golgi intermediate compartment",
  "gene_symbol": "TMED6"
}